{
  "gene_name": "ARF GTPase-activating protein GIT1",
  "gene": "UniProtKB:Q9Y2X7",
  "term_label": "postsynapse",
  "gene_symbol": "GIT1",
  "term_id": "GO:0098794"
}